oxidoreduction-driven active transmembrane transporter activity [GO:0015453] (molecular function) Definition: Primary active transport of a solute across a membrane, driven by exothermic flow of electrons from a reduced substrate to an oxidized substrate. Primary active transport is catalysis of the transport of a solute across a membrane, up the solute's concentration gradient, by binding the solute and undergoing a series of conformational changes. Transport works equally well in either direction and is driven by a primary energy source. Also known as: oxidoreduction-driven transporter Subtypes: cytochrome-c oxidase activity [GO:0004129], quinol-cytochrome-c reductase activity [GO:0008121], NADH dehydrogenase (ubiquinone) activity [GO:0008137], proton-translocating NAD(P)+ transhydrogenase activity [GO:0008750], GO:0009486, plastoquinol--plastocyanin reductase activity [GO:0009496], GO:0140571 Sources: GOC:mtg_transport, ISBN:0815340729, TC:3.D.-.-.- Relationships: is a type of primary active transmembrane transporter activity [GO:0015399]; has part GO:0016491